{
  "gene": "UniProtKB:P14867",
  "term_id": "GO:0032590",
  "gene_name": "Gamma-aminobutyric acid receptor subunit alpha-1",
  "term_label": "dendrite membrane",
  "gene_symbol": "GABRA1"
}